symbiont-mediated suppression of host natural killer cell activation [GO:0039672] (biological process) References: PMID:10799855 Relationships: is a type of symbiont-mediated perturbation of host natural killer cell mediated immune response [GO:0039671] Definition: A process in which a symbiont interferes with, inhibits or disrupts natural killer cell activation in the host. The host is defined as the larger of the organisms involved in a symbiotic interaction. Also known as: suppression by virus of host NK-cell activation, suppression by virus of host natural killer cell activation